{
  "gene_symbol": "CDH3",
  "gene_name": "Cadherin-3",
  "term_id": "GO:0045296",
  "term_label": "cadherin binding",
  "gene": "UniProtKB:P22223"
}